intracellularly cyclic nucleotide-activated monoatomic cation channel activity [GO:0005221] (molecular function) Definition: Enables the transmembrane transfer of a monoatomic cation by a channel that opens when intracellular cyclic nucleotide has been bound by the channel complex or one of its constituent parts. Also known as: intracellular cyclic nucleotide activated cation channel activity, intracellular cyclic nucleotide activated monoatomic cation channel activity, intracellular cyclic nucleotide-activated monoatomic cation channel activity Subtypes: GO:0005222, intracellularly cGMP-activated cation channel activity [GO:0005223] Sources: GOC:mtg_transport Relationships: is a type of intracellularly ligand-gated monoatomic ion channel activity [GO:0005217]; is a type of cyclic nucleotide-activated monoatomic ion channel activity [GO:0043855]; is_a ligand-gated monoatomic cation channel activity [GO:0099094]